{
  "gene": "UniProtKB:Q8WXI8",
  "gene_name": "C-type lectin domain family 4 member D",
  "gene_symbol": "CLEC4D",
  "term_id": "GO:0009897",
  "term_label": "external side of plasma membrane"
}